{
  "gene": "UniProtKB:P14778",
  "gene_name": "Interleukin-1 receptor type 1",
  "gene_symbol": "IL1R1",
  "term_id": "GO:0070498",
  "term_label": "interleukin-1-mediated signaling pathway"
}